{
  "gene_symbol": "SCRIB",
  "term_label": "protein kinase binding",
  "term_id": "GO:0019901",
  "gene": "UniProtKB:Q14160",
  "gene_name": "Protein scribble homolog"
}